{
  "term_id": "GO:0006888",
  "gene_name": "Trafficking protein particle complex subunit 5",
  "gene": "UniProtKB:Q8IUR0",
  "gene_symbol": "TRAPPC5",
  "term_label": "endoplasmic reticulum to Golgi vesicle-mediated transport"
}